{
  "gene": "UniProtKB:Q99963",
  "gene_name": "Endophilin-A3",
  "term_id": "GO:0006897",
  "gene_symbol": "SH3GL3",
  "term_label": "endocytosis"
}